{
  "gene": "UniProtKB:Q13148",
  "term_label": "RNA binding",
  "gene_name": "TAR DNA-binding protein 43",
  "gene_symbol": "TARDBP",
  "term_id": "GO:0003723"
}